{
  "term_label": "Unknown cellular component",
  "gene": "UniProtKB:Q8N4S7",
  "term_id": "UNKNOWN:0003",
  "gene_symbol": "PAQR4",
  "gene_name": "Progestin and adipoQ receptor family member 4"
}